peroxide sensor activity [GO:0140442] (molecular function) Relationships: is a type of molecular sensor activity [GO:0140299]; is part of response to hydrogen peroxide [GO:0042542] Definition: Binding to hydrogen peroxide (H2O2) and eliciting a change in the protein's activity in response to the intracellular level of that small molecule. References: PMID:20919928